{
  "gene_name": "Collectrin",
  "gene_symbol": "CLTRN",
  "term_label": "Unknown molecular function",
  "term_id": "UNKNOWN:0001",
  "gene": "UniProtKB:Q9HBJ8"
}